{
  "gene_symbol": "FCGR3A",
  "gene_name": "Low affinity immunoglobulin gamma Fc region receptor III-A",
  "gene": "UniProtKB:P08637",
  "term_label": "IgG receptor activity",
  "term_id": "GO:0019770"
}